promoter-enhancer loop anchoring activity [GO:0140585] (molecular function) Note: Note that GO does not separately defines enhancers, since this concept is very close to that of cis-regulatory elements. However the literature refers to 'promoter-enhancer loops' to describe loops that bring together cis-regulatory elements. Note also that while SO defines 'promoter' as the core promoter, here it is used to mean a cis-regulatory element. Relationships: is a type of chromatin loop anchoring activity [GO:0140587] References: PMID:32213323 Definition: Bridging together two cis-regulatory elements, colloquially referred to as promoters and/or enhancers, holding two loop anchors together to maintain a chromatin loop. Also known as: enhancer-promoter loop anchoring activity